{
  "gene_symbol": "TMEM170A",
  "gene": "UniProtKB:Q8WVE7",
  "term_label": "endoplasmic reticulum tubular network organization",
  "gene_name": "Transmembrane protein 170A",
  "term_id": "GO:0071786"
}